{
  "gene_symbol": "SCYGR4",
  "gene": "UniProtKB:A0A286YEV6",
  "term_id": "UNKNOWN:0001",
  "term_label": "Unknown molecular function",
  "gene_name": "Small cysteine and glycine repeat-containing protein 4"
}